{
  "gene_symbol": "MRGPRG-AS1",
  "term_label": "Unknown biological process",
  "gene_name": "Putative uncharacterized protein MRGPRG-AS1",
  "term_id": "UNKNOWN:0002",
  "gene": "UniProtKB:Q2M3A8"
}